{
  "gene_symbol": "TRGV4",
  "gene": "UniProtKB:A0A0C4DH28",
  "gene_name": "T cell receptor gamma variable 4",
  "term_label": "Unknown cellular component",
  "term_id": "UNKNOWN:0003"
}